sinus venosus formation [GO:0003237] (biological process) Definition: The developmental process pertaining to the initial formation of the sinus venosus from unspecified parts. The sinus venosus is a heart chamber attached to the atrium on the venous side of the embryonic heart. Relationships: is a type of cardiac chamber formation [GO:0003207]; is part of sinus venosus morphogenesis [GO:0003236] Sources: GOC:mtg_heart